{
  "term_id": "UNKNOWN:0003",
  "gene_name": "Required for meiotic nuclear division protein 1 homolog",
  "gene_symbol": "RMND1",
  "term_label": "Unknown cellular component",
  "gene": "UniProtKB:Q9NWS8"
}